{
  "term_label": "caveola",
  "gene": "UniProtKB:P16671",
  "gene_name": "Platelet glycoprotein 4",
  "term_id": "GO:0005901",
  "gene_symbol": "CD36"
}